{
  "term_id": "GO:0005007",
  "term_label": "fibroblast growth factor receptor activity",
  "gene_symbol": "FGFR4",
  "gene": "UniProtKB:P22455",
  "gene_name": "Fibroblast growth factor receptor 4"
}